{
  "gene_name": "Transmembrane protein 41A",
  "gene_symbol": "TMEM41A",
  "gene": "UniProtKB:Q96HV5",
  "term_id": "UNKNOWN:0002",
  "term_label": "Unknown biological process"
}